{
  "term_id": "UNKNOWN:0001",
  "term_label": "Unknown molecular function",
  "gene_name": "T-cell leukemia translocation-altered gene protein",
  "gene_symbol": "TCTA",
  "gene": "UniProtKB:P57738"
}